{
  "gene_symbol": "TRDJ1",
  "term_label": "Unknown biological process",
  "gene_name": "T cell receptor delta joining 1",
  "gene": "UniProtKB:A0A075B706",
  "term_id": "UNKNOWN:0002"
}